{
  "term_label": "synapse",
  "gene": "UniProtKB:O75309",
  "term_id": "GO:0045202",
  "gene_name": "Cadherin-16",
  "gene_symbol": "CDH16"
}